{
  "gene_name": "Leukocyte receptor cluster member 1",
  "gene_symbol": "LENG1",
  "gene": "UniProtKB:Q96BZ8",
  "term_label": "Unknown cellular component",
  "term_id": "UNKNOWN:0003"
}